negative regulation of small molecule metabolic process [GO:0062014] (biological process) Sources: GOC:vw Also known as: negative regulation of small molecule metabolism Relationships: is a type of negative regulation of metabolic process [GO:0009892]; is_a regulation of small molecule metabolic process [GO:0062012]; negatively regulates small molecule metabolic process [GO:0044281] Subtypes: negative regulation of gibberellin biosynthetic process [GO:0010373], negative regulation of penicillin catabolic process [GO:0033248], negative regulation of gluconeogenesis [GO:0045721], GO:0045753, GO:0045922, negative regulation of nucleoside metabolic process [GO:0045978], GO:0045980, negative regulation of purine nucleobase metabolic process [GO:0045982], negative regulation of pyrimidine nucleobase metabolic process [GO:0045984], negative regulation of ecdysteroid biosynthetic process [GO:0045997], negative regulation of vitamin metabolic process [GO:0046137], negative regulation of all-trans-retinyl-ester hydrolase, 11-cis retinol forming activity [GO:0062003], negative regulation of L-glutamine biosynthetic process [GO:0062133], negative regulation of bile acid biosynthetic process [GO:0070858], GO:0090206, negative regulation of (R)-mevalonic acid biosynthetic process [GO:0106108], negative regulation of UDP-N-acetylglucosamine biosynthetic process [GO:0106279], negative regulation of histidine biosynthetic process [GO:0120214], negative regulation of pyruvate decarboxylation to acetyl-CoA [GO:0160218], negative regulation of arginine catabolic process [GO:1900082], GO:1900178, negative regulation of xanthone-containing compound biosynthetic process [GO:1900184], negative regulation of penicillin biosynthetic process [GO:1900197], negative regulation of methane biosynthetic process from formic acid [GO:1900340], GO:1900380, negative regulation of alcohol catabolic process [GO:1900420], negative regulation of xylose catabolic process to ethanol [GO:1900516], negative regulation of emericellamide biosynthetic process [GO:1900659], negative regulation of emodin biosynthetic process [GO:1900665], negative regulation of endocrocin biosynthetic process [GO:1900668], negative regulation of fumonisin biosynthetic process [GO:1900684], negative regulation of gerfelin biosynthetic process [GO:1900687], negative regulation of o-orsellinic acid biosynthetic process [GO:1900699], GO:1900708, negative regulation of tensidol B biosynthetic process [GO:1900711], negative regulation of helvolic acid biosynthetic process [GO:1900841], negative regulation of monodictyphenone biosynthetic process [GO:1900844], negative regulation of naphtho-gamma-pyrone biosynthetic process [GO:1900847], negative regulation of pseurotin A biosynthetic process [GO:1900850], negative regulation of sarcinapterin biosynthetic process [GO:1900972], GO:1900975, negative regulation of tetrapyrrole biosynthetic process from glycine and succinyl-CoA [GO:1901414], negative regulation of ferulate catabolic process [GO:1901467], negative regulation of homoserine biosynthetic process [GO:1901711], GO:1901713, negative regulation of gamma-aminobutyric acid catabolic process [GO:1901716], negative regulation of indoleacetic acid biosynthetic process via tryptophan [GO:1901997], GO:1902006, negative regulation of fumagillin biosynthetic process [GO:1902091], negative regulation of alcohol biosynthetic process [GO:1902931], GO:1902987, GO:1903196, negative regulation of citrulline biosynthetic process [GO:1903249], negative regulation of ornithine catabolic process [GO:1903267], GO:1903455, negative regulation of glucose catabolic process to lactate via pyruvate [GO:1904024], negative regulation of ubiquinone biosynthetic process [GO:1904774], negative regulation of quinolinate biosynthetic process [GO:1904985], negative regulation of progesterone biosynthetic process [GO:2000183], GO:2000212, GO:2000225, GO:2000875, negative regulation of glycolytic fermentation to ethanol [GO:2001155], negative regulation of isopentenyl diphosphate biosynthetic process, mevalonate pathway [GO:2001211], GO:2001277 Definition: Any process that stops, prevents or reduces the frequency, rate or extent of a small molecule metabolic process.